cortical cytoskeleton organization [GO:0030865] (biological process) Definition: A process that is carried out at the cellular level which results in the assembly, arrangement of constituent parts, or disassembly of cytoskeletal structures in the cell cortex, i.e. just beneath the plasma membrane. Subtypes: cortical actin cytoskeleton organization [GO:0030866], cortical microtubule organization [GO:0043622], cytoskeletal matrix organization at active zone [GO:0048789] Also known as: cortical cytoskeleton organisation, cortical cytoskeleton organization and biogenesis Sources: GOC:dph, GOC:jl, GOC:mah Relationships: is a type of cytoskeleton organization [GO:0007010]